{
  "gene_symbol": "KRTAP10-6",
  "term_id": "UNKNOWN:0003",
  "term_label": "Unknown cellular component",
  "gene_name": "Keratin-associated protein 10-6",
  "gene": "UniProtKB:P60371"
}